{
  "gene_symbol": "DNAI4",
  "gene_name": "Dynein axonemal intermediate chain 4",
  "term_label": "dynein heavy chain binding",
  "gene": "UniProtKB:Q5VTH9",
  "term_id": "GO:0045504"
}